{
  "term_label": "sperm midpiece",
  "gene_symbol": "CD52",
  "gene_name": "CAMPATH-1 antigen",
  "gene": "UniProtKB:P31358",
  "term_id": "GO:0097225"
}